lsiRNA processing [GO:0010599] (biological process) Also known as: RNA interference, production of lsiRNA, primary lsiRNA processing, production of lsiRNA involved in RNA interference Definition: A process leading to the generation of a functional long small interfering RNA (lsiRNA). lsiRNAs are class of siRNAs 30 to 40 nt in length. lsiRNAs are induced by pathogen infection or under specific growth conditions. Relationships: is a type of siRNA processing [GO:0030422]; BFO_0000050 regulatory ncRNA-mediated post-transcriptional gene silencing [GO:0035194] References: PMID:18003861, PMID:20687832